{
  "term_id": "GO:0005737",
  "gene": "UniProtKB:O60260",
  "gene_symbol": "PRKN",
  "term_label": "cytoplasm",
  "gene_name": "E3 ubiquitin-protein ligase parkin"
}